{
  "term_label": "response to steroid hormone",
  "gene": "UniProtKB:P05412",
  "gene_symbol": "JUN",
  "term_id": "GO:0048545",
  "gene_name": "Transcription factor Jun"
}